{
  "gene_symbol": "MUC19",
  "gene": "UniProtKB:Q7Z5P9",
  "gene_name": "Mucin-19",
  "term_id": "UNKNOWN:0002",
  "term_label": "Unknown biological process"
}